{
  "gene_symbol": "KIF6",
  "gene": "UniProtKB:Q6ZMV9",
  "term_id": "GO:0005737",
  "term_label": "cytoplasm",
  "gene_name": "Kinesin-like protein KIF6"
}